epithelial cell type specification, open tracheal system [GO:0035153] (biological process) Also known as: tracheal cell type specification, tracheal epithelial cell type specification Definition: Allocation of epithelial cells within each migrating branch in an open tracheal system to distinct tracheal cell fates. During the migration phase each branch forms a well-defined number of cell types (including fusion cells, terminal cells and branch cells) at precise positions. Relationships: is_a cell fate specification [GO:0001708]; is part of open tracheal system development [GO:0007424] Subtypes: terminal cell fate specification, open tracheal system [GO:0035154], fusion cell fate specification [GO:0035156] References: PMID:10684581, PMID:11063940 Sources: GOC:mtg_sensu